response to docetaxel trihydrate [GO:1902519] (BP) Also known as: response to docetaxel Note: Note that this term is in the subset of terms that should not be used for direct manual annotation of gene products. It was created to be used for cross-referencing by other ontologies. Direct annotations to this term may be amended during annotation QC. References: PMID:23648065 Sources: GOC:TermGenie, GOC:dw Definition: Any process that results in a change in state or activity of a cell or an organism (in terms of movement, secretion, enzyme production, gene expression, etc.) as a result of a docetaxel trihydrate stimulus. Relationships: is a type of response to alcohol [GO:0097305]; is a type of response to ketone [GO:1901654]